double membrane vesicle viral factory assembly [GO:0140526] (biological process) Relationships: is a type of cellular component assembly [GO:0022607] References: PMID:32555292 Definition: A process that results in the assembly of a cytoplasmic viral factory consisting of a double-membrane bound vesicle.